{
  "gene_symbol": "BICD2",
  "gene": "UniProtKB:Q8TD16",
  "term_label": "Golgi apparatus",
  "gene_name": "Protein bicaudal D homolog 2",
  "term_id": "GO:0005794"
}